{
  "gene": "UniProtKB:P08833",
  "gene_name": "Insulin-like growth factor-binding protein 1",
  "term_label": "regulation of insulin-like growth factor receptor signaling pathway",
  "gene_symbol": "IGFBP1",
  "term_id": "GO:0043567"
}